saccharopine dehydrogenase activity [GO:0004753] (MF) Sources: GOC:mah Relationships: is a type of oxidoreductase activity, acting on the CH-NH group of donors, NAD or NADP as acceptor [GO:0016646] Also known as: lysine-2-oxoglutarate reductase activity, lysine-ketoglutarate reductase activity Definition: Catalysis of the cleavage of N6-(L-1,3-dicarboxypropyl)-L-lysine to release an amino acid (lysine or glutamate), with the concomitant reduction of an electron acceptor. Subtypes: GO:0004754, saccharopine dehydrogenase (NADP+, L-glutamate-forming) activity [GO:0004755], saccharopine dehydrogenase (NADP+, L-lysine-forming) activity [GO:0047130], saccharopine dehydrogenase (NAD+, L-glutamate-forming) activity [GO:0047131]